{
  "gene_symbol": "CHRNE",
  "gene": "UniProtKB:Q04844",
  "term_id": "GO:0005892",
  "term_label": "acetylcholine-gated channel complex",
  "gene_name": "Acetylcholine receptor subunit epsilon"
}